plasma membrane tubulation [GO:0097320] (biological process) Also known as: membrane tubulation, vesicle scission Relationships: is a type of plasma membrane organization [GO:0007009] References: PMID:15252009, PMID:20730103 Sources: GOC:BHF, GOC:pr Regulation: regulated by regulation of membrane tubulation [GO:1903525]; negatively regulated by negative regulation of membrane tubulation [GO:1903526]; positively regulated by GO:1903527 Definition: A membrane tubulation process occurring in a plasma membrane.